salivary gland histolysis [GO:0035070] (biological process) Definition: The stage-specific break down of the larval salivary glands during Drosophila metamorphosis, to allow replacement of larval structures by tissues and structures that form the adult fly. Relationships: is a type of salivary gland morphogenesis [GO:0007435]; is a type of post-embryonic animal morphogenesis [GO:0009886]; is a type of GO:0060033; is part of metamorphosis [GO:0007552]; is part of instar larval or pupal morphogenesis [GO:0048707] Also known as: salivary gland regression References: PMID:9409683 Sources: GOC:bf, GOC:dph, GOC:mtg_apoptosis